regulation of protein O-linked glycosylation [GO:1904098] (biological process) Definition: Any process that modulates the frequency, rate or extent of protein O-linked glycosylation. References: PMID:24509081 Sources: GOC:TermGenie, GO_REF:0000058 Also known as: regulation of protein amino acid O-linked glycosylation Relationships: is a type of regulation of glycoprotein biosynthetic process [GO:0010559]; RO_0002211 protein O-linked glycosylation [GO:0006493] Subtypes: GO:0010908, negative regulation of protein O-linked glycosylation [GO:1904099], positive regulation of protein O-linked glycosylation [GO:1904100]